{
  "term_label": "ubiquitin-like ligase-substrate adaptor activity",
  "term_id": "GO:1990756",
  "gene_name": "PRAME family member 14",
  "gene": "UniProtKB:Q5SWL7",
  "gene_symbol": "PRAMEF14"
}